{
  "gene": "UniProtKB:P38398",
  "gene_name": "Breast cancer type 1 susceptibility protein",
  "term_label": "double-strand break repair via homologous recombination",
  "gene_symbol": "BRCA1",
  "term_id": "GO:0000724"
}